cellular response to brefeldin A [GO:0071238] (biological process) Definition: Any process that results in a change in state or activity of a cell (in terms of movement, secretion, enzyme production, gene expression, etc.) as a result of a brefeldin A stimulus. Relationships: is_a response to brefeldin A [GO:0031001]; is a type of GO:0071236; is a type of cellular response to oxygen-containing compound [GO:1901701] Sources: GOC:mah